{
  "gene": "UniProtKB:P35244",
  "term_label": "damaged DNA binding",
  "gene_name": "Replication protein A 14 kDa subunit",
  "term_id": "GO:0003684",
  "gene_symbol": "RPA3"
}